postsynaptic intermediate filament cytoskeleton organization [GO:0099185] (biological process) Relationships: is a type of intermediate filament cytoskeleton organization [GO:0045104]; is a type of postsynaptic cytoskeleton organization [GO:0099188] Sources: GOC:dos Definition: A process that is carried out at the cellular level which results in the assembly, arrangement of constituent parts, or disassembly of cytoskeletal structures comprised of intermediate filament and their associated proteins in the postsynaptic cytoskeleton.